{
  "gene_symbol": "DCAF8L1",
  "gene": "UniProtKB:A6NGE4",
  "term_id": "GO:0005737",
  "gene_name": "DDB1- and CUL4-associated factor 8-like protein 1",
  "term_label": "cytoplasm"
}